{
  "gene_name": "Protein STPG4",
  "gene_symbol": "STPG4",
  "gene": "UniProtKB:Q8N801",
  "term_label": "histone binding",
  "term_id": "GO:0042393"
}